zygote elongation [GO:0080159] (biological process) Definition: The process in which the zygote irreversibly increases in size in one dimension after fertilization. An example of such a process is found in Arabidopsis thaliana. Relationships: is a type of unidimensional cell growth [GO:0009826]; is a type of embryonic morphogenesis [GO:0048598] Sources: GOC:tb